{
  "gene": "UniProtKB:Q6PXP3",
  "gene_symbol": "SLC2A7",
  "gene_name": "Solute carrier family 2, facilitated glucose transporter member 7",
  "term_label": "dehydroascorbic acid transport",
  "term_id": "GO:0070837"
}